{
  "term_id": "GO:0030031",
  "gene_symbol": "QRICH2",
  "gene": "UniProtKB:Q9H0J4",
  "gene_name": "Glutamine-rich protein 2",
  "term_label": "cell projection assembly"
}